{
  "term_label": "odorant binding",
  "gene_symbol": "OR5D3",
  "gene": "UniProtKB:A0A2R8Y4L6",
  "term_id": "GO:0005549",
  "gene_name": "Olfactory receptor"
}